{
  "gene": "UniProtKB:Q9H2U6",
  "term_id": "UNKNOWN:0003",
  "term_label": "Unknown cellular component",
  "gene_name": "Putative uncharacterized protein encoded by LINC00597",
  "gene_symbol": "LINC00597"
}